{
  "term_id": "UNKNOWN:0003",
  "gene_symbol": "GPR63",
  "gene_name": "Probable G-protein coupled receptor 63",
  "term_label": "Unknown cellular component",
  "gene": "UniProtKB:Q9BZJ6"
}